{
  "gene": "UniProtKB:Q16401",
  "gene_symbol": "PSMD5",
  "term_id": "UNKNOWN:0001",
  "term_label": "Unknown molecular function",
  "gene_name": "26S proteasome non-ATPase regulatory subunit 5"
}